{
  "term_id": "UNKNOWN:0001",
  "term_label": "Unknown molecular function",
  "gene_name": "High mobility group protein B2",
  "gene": "UniProtKB:P26583",
  "gene_symbol": "HMGB2"
}